{
  "gene_name": "Tripartite motif-containing protein 66",
  "term_id": "UNKNOWN:0002",
  "term_label": "Unknown biological process",
  "gene": "UniProtKB:O15016",
  "gene_symbol": "TRIM66"
}